{
  "gene_name": "Gap junction alpha-5 protein",
  "gene": "UniProtKB:P36382",
  "gene_symbol": "GJA5",
  "term_label": "connexin complex",
  "term_id": "GO:0005922"
}